{
  "gene_symbol": "HAPLN4",
  "term_id": "GO:0005615",
  "gene": "UniProtKB:Q86UW8",
  "gene_name": "Hyaluronan and proteoglycan link protein 4",
  "term_label": "extracellular space"
}